{
  "gene_symbol": "ZNF354A",
  "gene_name": "Zinc finger protein 354A",
  "term_label": "RNA polymerase II cis-regulatory region sequence-specific DNA binding",
  "term_id": "GO:0000978",
  "gene": "UniProtKB:O60765"
}